{
  "term_id": "GO:0034706",
  "gene_symbol": "SCNN1A",
  "gene": "UniProtKB:P37088",
  "term_label": "sodium channel complex",
  "gene_name": "Amiloride-sensitive sodium channel subunit alpha"
}